{
  "term_label": "nucleus",
  "gene_name": "DH domain-containing protein",
  "gene_symbol": "LOC107987545",
  "term_id": "GO:0005634",
  "gene": "UniProtKB:A0A2R8YFR7"
}